{
  "gene_symbol": "TF",
  "gene_name": "Serotransferrin",
  "term_id": "GO:0006826",
  "term_label": "iron ion transport",
  "gene": "UniProtKB:P02787"
}